{
  "gene_name": "Putative uncharacterized protein HSD52",
  "gene_symbol": "HSD52",
  "term_id": "UNKNOWN:0003",
  "gene": "UniProtKB:Q0P140",
  "term_label": "Unknown cellular component"
}